positive regulation of sulfur utilization [GO:0045883] (biological process) Sources: GOC:go_curators Definition: Any process that activates or increases the frequency, rate or extent of sulfur utilization. Relationships: is a type of regulation of sulfur utilization [GO:0006792]; is a type of GO:0032109; positively regulates sulfur utilization [GO:0006791] Also known as: positive regulation of sulphur utilization, up regulation of sulfur utilization, up-regulation of sulfur utilization, upregulation of sulfur utilization, activation of sulfur utilization, stimulation of sulfur utilization